{
  "gene_name": "Putative uncharacterized protein FLJ46204",
  "term_id": "UNKNOWN:0002",
  "gene": "UniProtKB:Q6ZRP5",
  "gene_symbol": "Q6ZRP5",
  "term_label": "Unknown biological process"
}